macropinocytic cup [GO:0070685] (cellular component) References: PMID:12538772, PMID:16968738, PMID:9044041 Definition: A cell projection that forms at the site of macropinocytosis, a form of endocytosis that results in the uptake of relatively large amounts of extracellular fluid. The macropinocytic cup membrane selectively excludes certain proteins, such as H36 or PM4C4 in Dictyostelium, and the underlying cytoskeleton is enriched in F-actin and coronin. Also known as: crown Relationships: is a type of plasma membrane bounded cell projection [GO:0120025]